butyryl-CoA biosynthetic process from acetyl-CoA [GO:0044579] (biological process) Definition: The chemical reactions and pathway resulting in the formation of butyryl-CoA, starting from acetyl-CoA. References: PMID:19539744 Sources: GOC:mengo_curators, GOC:tt Also known as: butyryl-CoA biosynthesis from acetyl-CoA Relationships: is a type of GO:0006084; is a type of butyryl-CoA biosynthetic process [GO:0044578] Regulation: regulated by regulation of butyryl-CoA biosynthetic process from acetyl-CoA [GO:1900494]; negatively regulated by negative regulation of butyryl-CoA biosynthetic process from acetyl-CoA [GO:1900495]; positively regulated by GO:1900496